{
  "term_id": "GO:0006635",
  "gene_name": "Enoyl-CoA delta isomerase 1, mitochondrial",
  "gene_symbol": "ECI1",
  "gene": "UniProtKB:P42126",
  "term_label": "fatty acid beta-oxidation"
}